Syp1 complex [GO:1990252] (cellular component) References: PMID:19713939 Sources: GOC:bhm Relationships: is a type of protein-containing complex [GO:0032991]; is part of clathrin-coated endocytic vesicle [GO:0045334] Definition: A protein complex that contributes to the endocytic process and bud growth in yeast. It is involved in the precise timing of actin assembly during endocytosis. Also known as: Syp1 dimer